host-mediated activation of viral transcription [GO:0043923] (biological process) Sources: GOC:jl Definition: A process in which a host organism initiates, promotes, or enhances the normal execution of viral transcription, the synthesis of either RNA on a template of DNA or DNA on a template of RNA. Also known as: positive regulation by host of viral transcription, positive regulation of viral transcription by host Subtypes: host-mediated activation of viral RNA-templated transcription [GO:0140181] Relationships: is_a GO:0043921; is a type of GO:0044794